cellular response to phenylalanine [GO:0071234] (BP) Definition: Any process that results in a change in state or activity of a cell (in terms of movement, secretion, enzyme production, gene expression, etc.) as a result of a phenylalanine stimulus. Sources: GOC:mah Relationships: is a type of cellular response to amino acid stimulus [GO:0071230]; is a type of response to phenylalanine [GO:0080053]; is a type of cellular response to nitrogen compound [GO:1901699]; is a type of GO:1901701